{
  "term_label": "Unknown biological process",
  "term_id": "UNKNOWN:0002",
  "gene": "UniProtKB:O15265",
  "gene_name": "Ataxin-7",
  "gene_symbol": "ATXN7"
}